{
  "gene": "UniProtKB:P10635",
  "term_label": "cytoplasm",
  "gene_name": "Cytochrome P450 2D6",
  "term_id": "GO:0005737",
  "gene_symbol": "CYP2D6"
}